{
  "gene_symbol": "VMA22",
  "gene_name": "Coiled-coil domain-containing protein 115",
  "term_id": "UNKNOWN:0002",
  "gene": "UniProtKB:Q96NT0",
  "term_label": "Unknown biological process"
}